{
  "term_label": "chromatin",
  "gene_symbol": "CHD6",
  "gene_name": "Chromodomain-helicase-DNA-binding protein 6",
  "gene": "UniProtKB:Q8TD26",
  "term_id": "GO:0000785"
}